ADP binding [GO:0043531] (molecular function) Also known as: adenosine 5'-diphosphate binding, adenosine diphosphate binding Regulation: negatively regulated by adenyl-nucleotide exchange factor activity [GO:0000774] Relationships: is a type of adenyl ribonucleotide binding [GO:0032559]; is a type of anion binding [GO:0043168] Definition: Binding to ADP, adenosine 5'-diphosphate. Sources: GOC:jl